mRNA binding [GO:0003729] (molecular function) Regulation: regulated by regulation of mRNA binding [GO:1902415]; RO_0002213 by positive regulation of mRNA binding [GO:1902416] Sources: GOC:kmv, GOC:pr, SO:0000234 Subtypes: mRNA 3'-UTR binding [GO:0003730], iron-responsive element binding [GO:0030350], triplet codon-amino acid adaptor activity [GO:0030533], selenocysteine insertion sequence binding [GO:0035368], mRNA 5'-UTR binding [GO:0048027], mRNA cap binding [GO:0098808], GO:1990715, GO:1990825 Also known as: base pairing with mRNA Definition: Binding to messenger RNA (mRNA), an intermediate molecule between DNA and protein. mRNA includes UTR and coding sequences, but does not contain introns. Relationships: is a type of RNA binding [GO:0003723]